abscisic acid transport [GO:0080168] (biological process) Definition: The directed movement of abscisic acid into, out of, within or between cells by means of some external agent such as a transporter or pore. References: PMID:20133881 Relationships: is_a monocarboxylic acid transport [GO:0015718]; is a type of GO:0015850; is a type of terpenoid transport [GO:0046865]